O-sialoglycoprotein catabolic process [GO:0045173] (biological process) References: PMID:8824323 Sources: GOC:go_curators Definition: The chemical reactions and pathways resulting in the breakdown of O-sialoglycoproteins, glycoproteins which contain sialic acid as one of their carbohydrates. They are often found on or in the cell or tissue membranes and participate in a variety of biological activities. Relationships: is a type of glycoprotein catabolic process [GO:0006516] Also known as: O-sialoglycoprotein breakdown, O-sialoglycoprotein catabolism, O-sialoglycoprotein degradation